programmed DNA elimination by elimination of internal DNA segments [GO:0140763] (biological process) Relationships: is_a programmed DNA elimination [GO:0031049] References: PMID:18708581 Definition: A programmed DNA elimination mechanism in which specific sequences, namely, internal eliminated sequences (IES) and breakage eliminated sequences (BES) are removed from the genome. This process is known to occur in ciliates.